{
  "term_label": "cytoplasm",
  "gene_symbol": "ALS2",
  "term_id": "GO:0005737",
  "gene_name": "Alsin",
  "gene": "UniProtKB:Q96Q42"
}